{
  "term_id": "GO:0008017",
  "gene_name": "G2 and S phase-expressed protein 1",
  "gene_symbol": "GTSE1",
  "gene": "UniProtKB:Q9NYZ3",
  "term_label": "microtubule binding"
}